{
  "term_label": "plasma membrane",
  "gene_name": "Melanotransferrin",
  "term_id": "GO:0005886",
  "gene": "UniProtKB:P08582",
  "gene_symbol": "MELTF"
}